{
  "term_label": "copper ion binding",
  "term_id": "GO:0005507",
  "gene_name": "Retina-specific copper amine oxidase",
  "gene": "UniProtKB:O75106",
  "gene_symbol": "AOC2"
}